{
  "gene_name": "Probable proline--tRNA ligase, mitochondrial",
  "gene": "UniProtKB:Q7L3T8",
  "term_id": "GO:0005739",
  "gene_symbol": "PARS2",
  "term_label": "mitochondrion"
}